{
  "term_label": "Unknown molecular function",
  "gene": "UniProtKB:Q9H579",
  "gene_symbol": "MROH8",
  "term_id": "UNKNOWN:0001",
  "gene_name": "Protein MROH8"
}